G-quadruplex unwinding activity [GO:0160225] (molecular function) References: PMID:1324186, PMID:26883636, PMID:34113828 Relationships: is a type of catalytic activity, acting on a nucleic acid [GO:0140640] Also known as: G-quadruplex resolving activity, G4 unwinding activity Definition: Unwinding G-quadruplex structures in nucleic acids. A G-quadruplex is a specialized structure formed in DNA/RNA when sequences rich in guanine (G) assemble into a unique four-stranded arrangement.